{
  "gene": "UniProtKB:P08603",
  "gene_symbol": "CFH",
  "gene_name": "Complement factor H",
  "term_id": "GO:0001851",
  "term_label": "complement component C3b binding"
}